establishment of protein localization to juxtaparanode region of axon [GO:0071206] (biological process) Definition: The directed movement of a protein to the juxtaparanode region of an axon. Also known as: establishment of protein localisation to juxtaparanode region of axon Sources: GOC:BHF, GOC:mah Relationships: is a type of establishment of protein localization [GO:0045184]